phosphatidylethanolamine transfer activity [GO:1904121] (molecular function) References: PMID:8606365 Sources: GOC:TermGenie, GO_REF:0000066 Definition: Removes phosphatidylethanolamine from a membrane or a monolayer lipid particle, transports it through the aqueous phase while protected in a hydrophobic pocket, and brings it to an acceptor membrane or lipid particle. Relationships: is a type of phospholipid transfer activity [GO:0120014] Also known as: phosphatidylethanolamine transporter activity, phosphatidylethanolamine carrier activity, intermembrane phosphatidylethanolamine transfer activity